{
  "term_label": "Unknown molecular function",
  "gene_name": "Transcription cofactor vestigial-like protein 1",
  "gene_symbol": "VGLL1",
  "gene": "UniProtKB:Q99990",
  "term_id": "UNKNOWN:0001"
}